ganglioside GT1b binding [GO:1905576] (molecular function) Definition: Binding to ganglioside GT1b. References: PMID:1454804 Sources: GOC:TermGenie, GO_REF:0000067 Relationships: is a type of carboxylic acid binding [GO:0031406]; is a type of ganglioside binding [GO:0035594]